{
  "gene_name": "Uncharacterized protein C1orf53",
  "gene_symbol": "C1orf53",
  "gene": "UniProtKB:Q5VUE5",
  "term_label": "Unknown cellular component",
  "term_id": "UNKNOWN:0003"
}